{
  "gene": "UniProtKB:O00192",
  "gene_symbol": "ARVCF",
  "term_label": "nucleus",
  "term_id": "GO:0005634",
  "gene_name": "Splicing regulator ARVCF"
}